{
  "gene_name": "Fibroblast growth factor 21",
  "gene_symbol": "FGF21",
  "term_id": "GO:0005737",
  "term_label": "cytoplasm",
  "gene": "UniProtKB:Q9NSA1"
}